regulation of cumulus cell differentiation [GO:0045592] (biological process) Relationships: is a type of regulation of epithelial cell differentiation [GO:0030856]; is a type of regulation of antral ovarian follicle growth [GO:2000387]; regulates cumulus cell differentiation [GO:0001549] Definition: Any process that modulates the frequency, rate or extent of ovarian cumulus cell differentiation. Sources: GOC:go_curators Subtypes: negative regulation of cumulus cell differentiation [GO:0045593], positive regulation of cumulus cell differentiation [GO:0045594] Also known as: regulation of ovarian cumulus cell differentiation